{
  "gene_name": "Angiomotin-like protein 2",
  "gene": "UniProtKB:Q9Y2J4",
  "term_id": "GO:0005886",
  "term_label": "plasma membrane",
  "gene_symbol": "AMOTL2"
}